{
  "term_label": "kinetochore",
  "gene_symbol": "TEX14",
  "term_id": "GO:0000776",
  "gene": "UniProtKB:Q8IWB6",
  "gene_name": "Inactive serine_threonine-protein kinase TEX14"
}